{
  "gene_symbol": "TBC1D3F",
  "gene": "UniProtKB:A6NER0",
  "term_label": "Unknown cellular component",
  "gene_name": "TBC1 domain family member 3F",
  "term_id": "UNKNOWN:0003"
}